{
  "term_id": "UNKNOWN:0003",
  "gene": "UniProtKB:Q8NDX6",
  "gene_name": "Zinc finger protein 740",
  "term_label": "Unknown cellular component",
  "gene_symbol": "ZNF740"
}